mesonephric smooth muscle tissue development [GO:0061214] (biological process) Sources: GOC:mtg_kidney_jan10 Relationships: is a type of kidney smooth muscle tissue development [GO:0072194]; is part of mesonephros development [GO:0001823] Definition: The process whose specific outcome is the progression of smooth muscle in the mesonephros over time, from its formation to the mature structure.